{
  "gene_name": "Protein Wnt-7a",
  "gene_symbol": "WNT7A",
  "gene": "UniProtKB:O00755",
  "term_label": "frizzled binding",
  "term_id": "GO:0005109"
}